histamine-gated chloride channel complex [GO:0019183] (cellular component) Definition: A protein complex that forms a transmembrane channel through which chloride ions may pass in response to histamine binding to the channel complex or one of its constituent parts. Sources: GOC:mah Relationships: is a type of GO:0034707; is a type of plasma membrane protein complex [GO:0098797]